{
  "gene": "UniProtKB:Q9H4T2",
  "gene_symbol": "ZSCAN16",
  "gene_name": "Zinc finger and SCAN domain-containing protein 16",
  "term_label": "Unknown cellular component",
  "term_id": "UNKNOWN:0003"
}